{
  "gene": "UniProtKB:O95376",
  "term_label": "cytoplasm",
  "gene_symbol": "ARIH2",
  "gene_name": "E3 ubiquitin-protein ligase ARIH2",
  "term_id": "GO:0005737"
}